{
  "gene": "UniProtKB:Q9ULQ0",
  "term_label": "protein-macromolecule adaptor activity",
  "term_id": "GO:0030674",
  "gene_name": "Striatin-interacting protein 2",
  "gene_symbol": "STRIP2"
}